{
  "term_id": "UNKNOWN:0001",
  "gene": "UniProtKB:C9JXX5",
  "gene_symbol": "FREY1",
  "gene_name": "Protein Frey 1",
  "term_label": "Unknown molecular function"
}